L-sorbose biosynthetic process [GO:0042849] (biological process) Definition: The chemical reactions and pathways resulting in the formation of L-sorbose, the L-enantiomer of the ketohexose xylo-2-hexulose. L-sorbose is formed by bacterial oxidation of sorbitol. Sources: ISBN:0198506732 Also known as: L-sorbose anabolism, L-sorbose biosynthesis, L-sorbose formation, L-sorbose synthesis Relationships: is_a GO:0019319